{
  "gene": "UniProtKB:A6NEL2",
  "gene_symbol": "SOWAHB",
  "term_label": "Unknown cellular component",
  "term_id": "UNKNOWN:0003",
  "gene_name": "Ankyrin repeat domain-containing protein SOWAHB"
}